{
  "gene": "UniProtKB:Q8NGZ3",
  "term_id": "GO:0050911",
  "term_label": "detection of chemical stimulus involved in sensory perception of smell",
  "gene_name": "Olfactory receptor 13G1",
  "gene_symbol": "OR13G1"
}